cellular response to trehalose stimulus [GO:0071327] (biological process) Sources: GOC:mah Definition: Any process that results in a change in state or activity of a cell (in terms of movement, secretion, enzyme production, gene expression, etc.) as a result of a trehalose stimulus. Relationships: is a type of response to trehalose [GO:0010353]; is a type of GO:0071324